{
  "term_id": "GO:0005615",
  "gene_name": "Angiopoietin-related protein 2",
  "gene_symbol": "ANGPTL2",
  "gene": "UniProtKB:Q9UKU9",
  "term_label": "extracellular space"
}